{
  "gene": "UniProtKB:Q6ZSA7",
  "term_label": "voltage-gated potassium channel activity",
  "gene_name": "Leucine-rich repeat-containing protein 55",
  "gene_symbol": "LRRC55",
  "term_id": "GO:0005249"
}